negative regulation of cell differentiation involved in embryonic placenta development [GO:0060806] (BP) Definition: Any process that decreases the rate, frequency or extent of cell differentiation that contributes to the progression of the placenta over time, from its initial condition to its mature state. Sources: GOC:dph, GOC:sdb_2009, GOC:tb Relationships: is a type of negative regulation of cell differentiation [GO:0045596]; is a type of regulation of cell differentiation involved in embryonic placenta development [GO:0060800]; is a type of GO:2000242; negatively regulates cell differentiation involved in embryonic placenta development [GO:0060706]